{
  "term_id": "GO:0000978",
  "gene_name": "Zinc finger protein ZIC 2",
  "gene": "UniProtKB:O95409",
  "gene_symbol": "ZIC2",
  "term_label": "RNA polymerase II cis-regulatory region sequence-specific DNA binding"
}